{
  "gene_symbol": "SYN1",
  "gene_name": "Synapsin-1",
  "gene": "UniProtKB:P17600",
  "term_id": "GO:0050808",
  "term_label": "synapse organization"
}